{
  "term_label": "binding of sperm to zona pellucida",
  "term_id": "GO:0007339",
  "gene": "UniProtKB:Q9BY14",
  "gene_symbol": "TEX101",
  "gene_name": "Testis-expressed protein 101"
}